{
  "term_id": "GO:0061172",
  "gene": "UniProtKB:Q8N957",
  "gene_symbol": "ANKFN1",
  "gene_name": "Ankyrin repeat and fibronectin type-III domain-containing protein 1",
  "term_label": "regulation of establishment of bipolar cell polarity"
}